{
  "term_label": "membrane",
  "gene_symbol": "SLC46A2",
  "term_id": "GO:0016020",
  "gene_name": "Thymic stromal cotransporter homolog",
  "gene": "UniProtKB:Q9BY10"
}